1,4-dihydroxy-2-naphthoate polyprenyltransferase activity [GO:0046428] (molecular function) Also known as: 1,4-dihydroxy-2-naphtoate prenyltransferase activity Relationships: is a type of prenyltransferase activity [GO:0004659] Definition: Catalysis of the reaction: 1,4-dihydroxy-2-naphthoate + an all-trans-polyprenyl diphosphate + H+ = a 2-demethylmenaquinol + CO2 + diphosphate. Sources: RHEA:26478